{
  "term_id": "GO:0010008",
  "gene": "UniProtKB:Q9ULQ1",
  "gene_symbol": "TPCN1",
  "gene_name": "Two pore channel protein 1",
  "term_label": "endosome membrane"
}